{
  "term_id": "GO:0016185",
  "gene_name": "Dynamin-2",
  "gene_symbol": "DNM2",
  "gene": "UniProtKB:P50570",
  "term_label": "synaptic vesicle budding from presynaptic endocytic zone membrane"
}